{
  "gene_symbol": "CCL5",
  "gene": "UniProtKB:P13501",
  "term_label": "chemokine activity",
  "term_id": "GO:0008009",
  "gene_name": "C-C motif chemokine 5"
}